regulation of aldosterone biosynthetic process [GO:0032347] (biological process) Relationships: is a type of regulation of ketone biosynthetic process [GO:0010566]; is a type of regulation of aldosterone metabolic process [GO:0032344]; is a type of regulation of steroid hormone biosynthetic process [GO:0090030]; is a type of regulation of alcohol biosynthetic process [GO:1902930]; regulates aldosterone biosynthetic process [GO:0032342] Sources: GOC:mah Subtypes: GO:0032348, GO:0032349 Definition: Any process that modulates the frequency, rate or extent of the chemical reactions and pathways resulting in the formation of aldosterone.